{
  "gene": "UniProtKB:O95447",
  "gene_symbol": "LCA5L",
  "term_id": "UNKNOWN:0001",
  "gene_name": "Lebercilin-like protein",
  "term_label": "Unknown molecular function"
}